positive regulation of positive chemotaxis [GO:0050927] (biological process) Definition: Any process that activates or increases the frequency, rate or extent of the directed movement of a motile cell or organism towards a higher concentration in a concentration gradient of a specific chemical. Sources: GOC:ai Also known as: up regulation of positive chemotaxis, up-regulation of positive chemotaxis, upregulation of positive chemotaxis, activation of positive chemotaxis, stimulation of positive chemotaxis Relationships: is a type of GO:0050921; is a type of GO:0050926; RO_0002213 positive chemotaxis [GO:0050918] Subtypes: induction of positive chemotaxis [GO:0050930], positive regulation of positive chemotaxis to cAMP [GO:0061122]